{
  "term_label": "structural constituent of chromatin",
  "gene_symbol": "H2AC12",
  "gene_name": "Histone H2A type 1-H",
  "term_id": "GO:0030527",
  "gene": "UniProtKB:Q96KK5"
}